translation release factor activity, codon nonspecific [GO:0016150] (MF) Sources: ISBN:0198547684 Relationships: is a type of translation release factor activity [GO:0003747] Definition: A translation release factor that is not specific to particular codons; binds to guanine nucleotides.